smooth muscle relaxation of the bladder outlet [GO:0060085] (biological process) Relationships: is a type of relaxation of smooth muscle [GO:0044557]; is a type of GO:0045986; is part of micturition [GO:0060073] References: PMID:15827347 Sources: GOC:dph Also known as: synaptic transmission involved in urination Definition: A process in which the extent of smooth muscle contraction is reduced in the bladder outlet that contributes to the expulsion of urine from the body.